{
  "gene": "UniProtKB:P59534",
  "term_id": "GO:0033038",
  "gene_symbol": "TAS2R39",
  "term_label": "bitter taste receptor activity",
  "gene_name": "Taste receptor type 2 member 39"
}